{
  "gene": "UniProtKB:Q9UKF6",
  "gene_symbol": "CPSF3",
  "term_id": "GO:0006398",
  "term_label": "mRNA 3'-end processing by stem-loop binding and cleavage",
  "gene_name": "Cleavage and polyadenylation specificity factor subunit 3"
}